{
  "gene": "UniProtKB:P0DP23",
  "gene_symbol": "CALM1",
  "term_id": "GO:0005509",
  "term_label": "calcium ion binding",
  "gene_name": "Calmodulin-1"
}